{
  "gene_name": "Retinol dehydrogenase 16",
  "term_label": "steroid metabolic process",
  "gene_symbol": "RDH16",
  "gene": "UniProtKB:O75452",
  "term_id": "GO:0008202"
}